{
  "gene_symbol": "GRM2",
  "gene_name": "Metabotropic glutamate receptor 2",
  "term_label": "group II metabotropic glutamate receptor activity",
  "gene": "UniProtKB:Q14416",
  "term_id": "GO:0001641"
}